{
  "gene": "UniProtKB:Q9Y222",
  "gene_name": "Cyclin-D-binding Myb-like transcription factor 1",
  "term_id": "GO:0000981",
  "gene_symbol": "DMTF1",
  "term_label": "DNA-binding transcription factor activity, RNA polymerase II-specific"
}